{
  "term_label": "Unknown biological process",
  "gene": "UniProtKB:Q58FG0",
  "gene_name": "Putative heat shock protein HSP 90-alpha A5",
  "term_id": "UNKNOWN:0002",
  "gene_symbol": "HSP90AA5P"
}